{
  "term_id": "GO:0005794",
  "gene": "UniProtKB:Q8NC42",
  "term_label": "Golgi apparatus",
  "gene_name": "E3 ubiquitin-protein ligase RNF149",
  "gene_symbol": "RNF149"
}